{
  "gene": "UniProtKB:P35346",
  "gene_symbol": "SSTR5",
  "term_id": "GO:0043005",
  "gene_name": "Somatostatin receptor type 5",
  "term_label": "neuron projection"
}